RNA nucleotide insertion [GO:0070705] (biological process) Definition: The modification of an RNA molecule by insertion of one or more nucleotides. Relationships: is a type of RNA modification [GO:0009451] Sources: GOC:cb, GOC:mah Subtypes: cotranscriptional mitochondrial rRNA nucleotide insertion [GO:0002110], RNA dinucleotide insertion [GO:0070707], RNA cytidine insertion [GO:0070708], GO:0070709